{
  "gene": "UniProtKB:Q86UB9",
  "term_label": "Unknown biological process",
  "gene_symbol": "TMEM135",
  "gene_name": "Transmembrane protein 135",
  "term_id": "UNKNOWN:0002"
}